regulation of localization [GO:0032879] (biological process) Definition: Any process that modulates the frequency, rate or extent of any process in which a cell, a substance, or a cellular entity is transported to, or maintained in, a specific location. Subtypes: GO:0032880, regulation of transport [GO:0051049], GO:0051282, Wnt signaling pathway, regulating spindle positioning [GO:0060069], regulation of exocyst localization [GO:0060178], regulation of cellular localization [GO:0060341], regulation of metaphase plate congression [GO:0090235], GO:0106020, regulation of interphase mitotic telomere clustering [GO:0110065], regulation of chromosome attachment to the nuclear envelope [GO:0120264], regulation of receptor localization to synapse [GO:1902683], GO:1902872, regulation of mitotic telomere tethering at nuclear periphery [GO:1904536], regulation of intracellular mRNA localization [GO:1904580], regulation of telomerase RNA localization to Cajal body [GO:1904872], GO:1904910, regulation of establishment of protein-containing complex localization to telomere [GO:1904913], regulation of lipid localization [GO:1905952], regulation of defense response by callose deposition [GO:2000071], regulation of synaptic vesicle clustering [GO:2000807] Sources: GOC:mah Also known as: regulation of localisation Relationships: is a type of regulation of biological process [GO:0050789]; regulates localization [GO:0051179]